positive regulation of keratinocyte apoptotic process [GO:1902174] (biological process) Definition: Any process that activates or increases the frequency, rate or extent of keratinocyte apoptotic process. References: PMID:18938133 Sources: GOC:BHF, GOC:TermGenie, GOC:mtg_apoptosis, GOC:rl Also known as: up regulation of keratinocyte apoptotic process, up-regulation of keratinocyte apoptotic process, upregulation of keratinocyte apoptotic process, activation of keratinocyte apoptosis, activation of keratinocyte apoptotic process, positive regulation of keratinocyte apoptosis, up regulation of keratinocyte apoptosis, up-regulation of keratinocyte apoptosis, upregulation of keratinocyte apoptosis Relationships: is a type of regulation of keratinocyte apoptotic process [GO:1902172]; is a type of positive regulation of epithelial cell apoptotic process [GO:1904037]; positively regulates keratinocyte apoptotic process [GO:0097283]